negative regulation of dense core granule exocytosis [GO:1905414] (BP) Also known as: down regulation of dense core granule exocytosis, down regulation of dense core vesicle exocytosis, down-regulation of dense core granule exocytosis, down-regulation of dense core vesicle exocytosis, downregulation of dense core granule exocytosis, downregulation of dense core vesicle exocytosis, negative regulation of dense core vesicle exocytosis, inhibition of dense core granule exocytosis, inhibition of dense core vesicle exocytosis Relationships: is a type of negative regulation of calcium ion-dependent exocytosis [GO:0045955]; is a type of regulation of dense core granule exocytosis [GO:1905413]; negatively regulates dense core granule exocytosis [GO:1990504] Definition: Any process that stops, prevents or reduces the frequency, rate or extent of dense core granule exocytosis. Sources: GOC:PARL, GOC:TermGenie, GOC:bf, GO_REF:0000058